{
  "term_id": "UNKNOWN:0001",
  "term_label": "Unknown molecular function",
  "gene_symbol": "DNAAF2",
  "gene": "UniProtKB:Q9NVR5",
  "gene_name": "Protein kintoun"
}